animal organ regeneration [GO:0031100] (BP) Relationships: is a type of regeneration [GO:0031099]; is a type of animal organ development [GO:0048513] Subtypes: liver regeneration [GO:0097421], pancreas regeneration [GO:1990798] Sources: GOC:mah Definition: The regrowth of a lost or destroyed animal organ.